{
  "gene_name": "Isopentenyl-diphosphate delta-isomerase 2",
  "term_id": "GO:0004452",
  "term_label": "isopentenyl-diphosphate delta-isomerase activity",
  "gene_symbol": "IDI2",
  "gene": "UniProtKB:Q9BXS1"
}